histone H2BK5 acetyltransferase activity [GO:0044014] (molecular function) Also known as: histone acetylase activity (H2B-K5 specific), histone acetyltransferase activity (H2B-K5 specific), histone lysine N-acetyltransferase activity (H2B-K5 specific) References: PMID:18552846 Definition: Catalysis of the reaction: acetyl-CoA + histone H2B L-lysine (position 5) = CoA + histone H2B N6-acetyl-L-lysine (position 5). Relationships: is a type of histone H2B acetyltransferase activity [GO:0044013] Note: Note that the residue position corresponds to the canonical human H2B histone (UniProtKB:P62807); the N-terminus of histone H2B is divergent across eukaryotes; make sure that the paper clearly references the human protein for the position of this modification to use this term. Residue 1 is the first residue following removal of the initiating Methionine (Met). Note that each histone is encoded by multiple genes, and sequences may vary across different genes within an organism.